{
  "gene": "UniProtKB:Q9UNP9",
  "gene_symbol": "PPIE",
  "term_id": "GO:0016018",
  "gene_name": "Peptidyl-prolyl cis-trans isomerase E",
  "term_label": "cyclosporin A binding"
}